alphaIIb-beta3 integrin-fibronectin-tissue transglutaminase complex [GO:0071090] (cellular component) Definition: A protein complex that consists of an alphaIIb-beta3 integrin complex bound to fibronectin and tissue transglutaminase. Also known as: ITGA2b-ITGB3-FN1-TGM2 complex References: PMID:10684262 Relationships: is a type of plasma membrane protein complex [GO:0098797]; is a type of GO:1902494